{
  "term_id": "GO:0042101",
  "gene": "UniProtKB:Q6PIZ9",
  "gene_name": "T-cell receptor-associated transmembrane adapter 1",
  "term_label": "T cell receptor complex",
  "gene_symbol": "TRAT1"
}